{
  "term_id": "GO:0016020",
  "gene": "UniProtKB:Q9H2Y7",
  "gene_name": "Zinc finger protein 106",
  "term_label": "membrane",
  "gene_symbol": "ZNF106"
}